{
  "gene_name": "Protein bicaudal D homolog 2",
  "gene": "UniProtKB:Q8TD16",
  "gene_symbol": "BICD2",
  "term_id": "GO:0034067",
  "term_label": "protein localization to Golgi apparatus"
}